{
  "term_id": "UNKNOWN:0003",
  "gene_symbol": "PRB3",
  "gene_name": "Basic salivary proline-rich protein 3",
  "gene": "UniProtKB:Q04118",
  "term_label": "Unknown cellular component"
}